glucosamine-6-phosphate deaminase activity [GO:0004342] (molecular function) Definition: Catalysis of the reaction: D-glucosamine 6-phosphate + H2O = beta-D-fructose 6-phosphate + NH4. Sources: EC:3.5.99.6, RHEA:12172 Also known as: glucosaminephosphate isomerase, 2-amino-2-deoxy-D-glucose-6-phosphate aminohydrolase (ketol isomerizing), GlcN6P deaminase activity, aminodeoxyglucosephosphate isomerase activity, glucosamine phosphate deaminase activity, glucosamine-6-phosphate isomerase activity, phosphoglucosamine isomerase activity, phosphoglucosaminisomerase activity Relationships: is a type of deaminase activity [GO:0019239]